positive regulation of 1-phosphatidyl-1D-myo-inositol 4,5-bisphosphate biosynthetic process [GO:1902648] (biological process) Definition: Any process that activates or increases the frequency, rate or extent of 1-phosphatidyl-1D-myo-inositol 4,5-bisphosphate biosynthetic process. Relationships: is a type of positive regulation of phosphatidylinositol biosynthetic process [GO:0010513]; is a type of regulation of 1-phosphatidyl-1D-myo-inositol 4,5-bisphosphate biosynthetic process [GO:1902646]; positively regulates 1-phosphatidyl-1D-myo-inositol 4,5-bisphosphate biosynthetic process [GO:1902635] Also known as: positive regulation of 1-phosphatidyl-1D-myo-inositol 4,5-bisphosphate anabolism, positive regulation of 1-phosphatidyl-1D-myo-inositol 4,5-bisphosphate biosynthesis, positive regulation of 1-phosphatidyl-1D-myo-inositol 4,5-bisphosphate formation, positive regulation of 1-phosphatidyl-1D-myo-inositol 4,5-bisphosphate synthesis, up regulation of 1-phosphatidyl-1D-myo-inositol 4,5-bisphosphate anabolism, up regulation of 1-phosphatidyl-1D-myo-inositol 4,5-bisphosphate biosynthesis, up regulation of 1-phosphatidyl-1D-myo-inositol 4,5-bisphosphate biosynthetic process, up regulation of 1-phosphatidyl-1D-myo-inositol 4,5-bisphosphate formation, up regulation of 1-phosphatidyl-1D-myo-inositol 4,5-bisphosphate synthesis, up-regulation of 1-phosphatidyl-1D-myo-inositol 4,5-bisphosphate anabolism, up-regulation of 1-phosphatidyl-1D-myo-inositol 4,5-bisphosphate biosynthesis, up-regulation of 1-phosphatidyl-1D-myo-inositol 4,5-bisphosphate biosynthetic process, up-regulation of 1-phosphatidyl-1D-myo-inositol 4,5-bisphosphate formation, up-regulation of 1-phosphatidyl-1D-myo-inositol 4,5-bisphosphate synthesis, upregulation of 1-phosphatidyl-1D-myo-inositol 4,5-bisphosphate anabolism, upregulation of 1-phosphatidyl-1D-myo-inositol 4,5-bisphosphate biosynthesis, upregulation of 1-phosphatidyl-1D-myo-inositol 4,5-bisphosphate biosynthetic process, upregulation of 1-phosphatidyl-1D-myo-inositol 4,5-bisphosphate formation, upregulation of 1-phosphatidyl-1D-myo-inositol 4,5-bisphosphate synthesis, activation of 1-phosphatidyl-1D-myo-inositol 4,5-bisphosphate anabolism, activation of 1-phosphatidyl-1D-myo-inositol 4,5-bisphosphate biosynthesis, activation of 1-phosphatidyl-1D-myo-inositol 4,5-bisphosphate biosynthetic process, activation of 1-phosphatidyl-1D-myo-inositol 4,5-bisphosphate formation, activation of 1-phosphatidyl-1D-myo-inositol 4,5-bisphosphate synthesis References: PMID:22562153 Sources: GOC:TermGenie, GOC:di, GO_REF:0000058